DIBOA-glucoside oxygenase activity [GO:0102717] (molecular function) Sources: EC:1.14.11.59, GOC:pz Definition: Catalysis of the reaction: DIBOA-beta-D-glucoside + O2 + 2-oxoglutarate = TRIBOA-beta-D-glucoside + succinate + carbon dioxide. Relationships: is a type of oxidoreductase activity, acting on paired donors, with incorporation or reduction of molecular oxygen, with 2-oxoglutarate as one donor, and the other dehydrogenated [GO:0050498]